cellular response to metal ion [GO:0071248] (biological process) Definition: Any process that results in a change in state or activity of a cell (in terms of movement, secretion, enzyme production, gene expression, etc.) as a result of a metal ion stimulus. Sources: GOC:mah Also known as: cellular response to metal, cellular response to heavy metal Relationships: is a type of response to metal ion [GO:0010038]; is a type of cellular response to chemical stimulus [GO:0070887] Subtypes: GO:0035865, cellular response to aluminum ion [GO:0071275], GO:0071276, GO:0071277, cellular response to cesium ion [GO:0071278], cellular response to cobalt ion [GO:0071279], cellular response to copper ion [GO:0071280], cellular response to iron ion [GO:0071281], cellular response to lead ion [GO:0071284], cellular response to lithium ion [GO:0071285], cellular response to magnesium ion [GO:0071286], GO:0071287, cellular response to mercury ion [GO:0071288], cellular response to nickel ion [GO:0071289], cellular response to platinum ion [GO:0071290], cellular response to selenium ion [GO:0071291], GO:0071292, cellular response to tellurium ion [GO:0071293], cellular response to zinc ion [GO:0071294], GO:1904312